cell migration involved in prostatic bud elongation [GO:0060518] (biological process) References: PMID:18977204 Sources: GOC:dph Relationships: is a type of epithelial cell migration [GO:0010631]; is part of primary prostatic bud elongation [GO:0060516] Definition: The orderly movement of epithelial cells from one site to another contributing to the elongation of the primary prostatic bud.